{
  "gene_symbol": "AKT3",
  "gene": "UniProtKB:Q9Y243",
  "term_id": "GO:0043066",
  "term_label": "negative regulation of apoptotic process",
  "gene_name": "RAC-gamma serine_threonine-protein kinase"
}